{
  "gene_name": "Frizzled-5",
  "gene_symbol": "FZD5",
  "term_label": "Wnt-protein binding",
  "term_id": "GO:0017147",
  "gene": "UniProtKB:Q13467"
}